{
  "term_id": "GO:0004222",
  "gene": "UniProtKB:Q9UKP4",
  "term_label": "metalloendopeptidase activity",
  "gene_name": "A disintegrin and metalloproteinase with thrombospondin motifs 7",
  "gene_symbol": "ADAMTS7"
}